trophoblast giant cell differentiation [GO:0060707] (biological process) References: PMID:16269175 Sources: GOC:dph Definition: The process in which a relatively unspecialized cell acquires specialized features of a trophoblast giant cell of the placenta. Trophoblast giant cells are the cell of the placenta that line the maternal decidua. Relationships: is_a cell differentiation involved in embryonic placenta development [GO:0060706]